{
  "gene_name": "Chorionic somatomammotropin hormone 2",
  "term_label": "response to nutrient levels",
  "gene_symbol": "CSH2",
  "gene": "UniProtKB:P0DML3",
  "term_id": "GO:0031667"
}